{
  "term_id": "GO:0007218",
  "term_label": "neuropeptide signaling pathway",
  "gene": "UniProtKB:P30872",
  "gene_symbol": "SSTR1",
  "gene_name": "Somatostatin receptor type 1"
}